megakaryocyte development [GO:0035855] (biological process) Also known as: megakaryocyte cell development Relationships: is a type of myeloid cell development [GO:0061515]; is part of megakaryocyte differentiation [GO:0030219] Definition: The process whose specific outcome is the progression of a megakaryocyte cell over time, from its formation to the mature structure. Megakaryocyte development does not include the steps involved in committing a cell to a megakaryocyte fate. A megakaryocyte is a giant cell 50 to 100 micron in diameter, with a greatly lobulated nucleus, found in the bone marrow. Sources: CL:0000556, GOC:BHF, GOC:vk